{
  "term_id": "GO:0005912",
  "gene": "UniProtKB:Q9UQB3",
  "term_label": "adherens junction",
  "gene_symbol": "CTNND2",
  "gene_name": "Catenin delta-2"
}